apolipoprotein A-I binding [GO:0034186] (MF) Sources: GOC:BHF, GOC:rl Relationships: is a type of apolipoprotein binding [GO:0034185] Definition: Binding to apolipoprotein A-I.